substrate-dependent cell migration, cell extension [GO:0006930] (biological process) Definition: The formation of a cell surface protrusion, such as a lamellipodium or filopodium, at the leading edge of a migrating cell. Relationships: is_a GO:0120031; is part of substrate-dependent cell migration [GO:0006929] Also known as: substrate-bound cell migration, cell extension References: PMID:11944043, PMID:14657486 Sources: ISBN:0815316194